(17Z)-protosta-17(20),24-dien-3beta-ol catabolic process [GO:1900580] (biological process) Sources: GOC:TermGenie, GOC:di Also known as: (17Z)-protosta-17(20),24-dien-3beta-ol breakdown, (17Z)-protosta-17(20),24-dien-3beta-ol catabolism, (17Z)-protosta-17(20),24-dien-3beta-ol degradation Definition: The chemical reactions and pathways resulting in the breakdown of (17Z)-protosta-17(20),24-dien-3beta-ol. Relationships: is a type of steroid catabolic process [GO:0006706]; is a type of triterpenoid catabolic process [GO:0016105]; is a type of alcohol catabolic process [GO:0046164]; is a type of GO:0090487; is a type of secondary alcohol metabolic process [GO:1902652]